cytoplasmic RNA surveillance [GO:0071026] (biological process) Definition: The set of processes involved in identifying and degrading defective or aberrant RNAs within the cytoplasm. Subtypes: mitochondrial RNA surveillance [GO:2000827] References: PMID:18644474 Sources: GOC:dgf, GOC:krc Also known as: cytoplasmic RNA quality control, cytoplasmic aberrant RNA catabolic process Relationships: is a type of RNA surveillance [GO:0071025]; occurs in GO:0005737